{
  "gene_symbol": "GPR119",
  "term_id": "GO:0005886",
  "gene": "UniProtKB:Q8TDV5",
  "term_label": "plasma membrane",
  "gene_name": "Glucose-dependent insulinotropic receptor"
}